cellular response to histidine [GO:0071232] (biological process) Definition: Any process that results in a change in state or activity of a cell (in terms of movement, secretion, enzyme production, gene expression, etc.) as a result of a histidine stimulus. Sources: GOC:mah Relationships: is a type of cellular response to amino acid stimulus [GO:0071230]; is a type of response to histidine [GO:0080052]; is a type of GO:1901699; is a type of cellular response to oxygen-containing compound [GO:1901701]